{
  "gene": "UniProtKB:O95793",
  "term_label": "cytoplasmic stress granule",
  "gene_name": "Double-stranded RNA-binding protein Staufen homolog 1",
  "gene_symbol": "STAU1",
  "term_id": "GO:0010494"
}